{
  "gene": "UniProtKB:O15552",
  "gene_name": "Free fatty acid receptor 2",
  "term_label": "plasma membrane",
  "gene_symbol": "FFAR2",
  "term_id": "GO:0005886"
}